{
  "gene_name": "Protein FAM177A1",
  "gene_symbol": "FAM177A1",
  "term_label": "Unknown molecular function",
  "gene": "UniProtKB:Q8N128",
  "term_id": "UNKNOWN:0001"
}